negative regulation of steroid hormone biosynthetic process [GO:0090032] (BP) Definition: Any process that decreases the frequency, rate or extent of the chemical reactions and pathways resulting in the formation of steroid hormones,compounds with a 1, 2, cyclopentanoperhydrophenanthrene nucleus that act as hormones. Relationships: is a type of negative regulation of steroid biosynthetic process [GO:0010894]; is a type of negative regulation of hormone biosynthetic process [GO:0032353]; is a type of regulation of steroid hormone biosynthetic process [GO:0090030] Subtypes: negative regulation of brassinosteroid biosynthetic process [GO:0010423], negative regulation of glucocorticoid biosynthetic process [GO:0031947], negative regulation of aldosterone biosynthetic process [GO:0032348], negative regulation of ecdysteroid biosynthetic process [GO:0045997] Sources: GOC:dph, GOC:tb